{
  "term_id": "GO:0005886",
  "term_label": "plasma membrane",
  "gene": "UniProtKB:P14616",
  "gene_name": "Insulin receptor-related protein",
  "gene_symbol": "INSRR"
}